{
  "term_label": "mitochondrion",
  "gene_name": "Thioredoxin-related transmembrane protein 2",
  "term_id": "GO:0005739",
  "gene": "UniProtKB:Q9Y320",
  "gene_symbol": "TMX2"
}